{
  "term_id": "GO:0046488",
  "term_label": "phosphatidylinositol metabolic process",
  "gene_name": "1-phosphatidylinositol 4,5-bisphosphate phosphodiesterase gamma-1",
  "gene_symbol": "PLCG1",
  "gene": "UniProtKB:P19174"
}